{
  "gene_name": "Uncharacterized protein C1orf131",
  "gene_symbol": "C1orf131",
  "term_id": "UNKNOWN:0003",
  "term_label": "Unknown cellular component",
  "gene": "UniProtKB:Q8NDD1"
}